L-glutamate uniporter activity [GO:0140788] (molecular function) Definition: Catalysis of the active transport of a L-glutamate across a membrane by a mechanism involving conformational change, where energy for active transport is derived from membrane potential if the solute is charged. Relationships: is a type of L-glutamate transmembrane transporter activity [GO:0005313]; is a type of membrane potential driven uniporter activity [GO:0022810] Also known as: glutamate uniporter activity References: PMID:27133463, PMID:29642010